{
  "gene_name": "Alpha-actinin-3",
  "term_label": "plasma membrane",
  "gene_symbol": "ACTN3",
  "gene": "UniProtKB:Q08043",
  "term_id": "GO:0005886"
}